{
  "term_id": "UNKNOWN:0002",
  "gene_symbol": "ERVK-25",
  "term_label": "Unknown biological process",
  "gene": "UniProtKB:P63136",
  "gene_name": "Endogenous retrovirus group K member 25 Pol protein"
}